{
  "gene_name": "Ski oncogene",
  "gene": "UniProtKB:P12755",
  "term_label": "RNA polymerase II cis-regulatory region sequence-specific DNA binding",
  "term_id": "GO:0000978",
  "gene_symbol": "SKI"
}